L-glutamate N-acetyltransferase activity [GO:0004042] (molecular function) Sources: RHEA:24292 Relationships: is a type of L-amino-acid N-acetyltransferase activity [GO:0140085] Definition: Catalysis of the reaction: L-glutamate + acetyl-CoA = N-acetyl-L-glutamate + CoA + H+. Also known as: N-acetylglutamate synthase activity, amino-acid N-acetyltransferase activity, acetyl-CoA:L-glutamate N-acetyltransferase activity, AGAS, acetylglutamate acetylglutamate synthetase activity, amino acid acetyltransferase activity